liquid clearance, open tracheal system [GO:0035002] (biological process) Relationships: is a type of epithelial fluid transport [GO:0042045]; is part of open tracheal system development [GO:0007424] Also known as: tracheal liquid clearance References: PMID:12571352 Sources: GOC:mtg_sensu Definition: The clearance of liquid from the epithelial tubes of an open tracheal system, shortly before the emergence of the larva, to generate an air-filled tubule system.